negative regulation of cell-substrate junction organization [GO:0150118] (biological process) Definition: Any process that stops, prevents or reduces the frequency, rate or extent of cell-substrate junction organization. Sources: GOC:aruk Relationships: is a type of negative regulation of cellular component organization [GO:0051129]; is a type of regulation of cell-substrate junction organization [GO:0150116]; negatively regulates cell-substrate junction organization [GO:0150115] Subtypes: negative regulation of focal adhesion assembly [GO:0051895], GO:0120184